{
  "gene": "UniProtKB:Q9NRJ3",
  "term_id": "GO:0005615",
  "gene_name": "C-C motif chemokine 28",
  "gene_symbol": "CCL28",
  "term_label": "extracellular space"
}